{
  "gene_name": "Spastin",
  "gene": "UniProtKB:Q9UBP0",
  "gene_symbol": "SPAST",
  "term_id": "GO:0008568",
  "term_label": "microtubule severing ATPase activity"
}